{
  "term_id": "UNKNOWN:0002",
  "gene": "UniProtKB:Q5TA78",
  "gene_name": "Late cornified envelope protein 4A",
  "gene_symbol": "LCE4A",
  "term_label": "Unknown biological process"
}